{
  "term_label": "Unknown molecular function",
  "gene_symbol": "FAM98A",
  "gene_name": "Protein FAM98A",
  "term_id": "UNKNOWN:0001",
  "gene": "UniProtKB:Q8NCA5"
}